{
  "gene_symbol": "YIPF5",
  "gene": "UniProtKB:Q969M3",
  "term_id": "UNKNOWN:0001",
  "term_label": "Unknown molecular function",
  "gene_name": "Protein YIPF5"
}